positive regulation of sodium ion transmembrane transport [GO:1902307] (biological process) Also known as: positive regulation of sodium ion membrane transport, up regulation of sodium ion membrane transport, up regulation of sodium ion transmembrane transport, up-regulation of sodium ion membrane transport, up-regulation of sodium ion transmembrane transport, upregulation of sodium ion membrane transport, upregulation of sodium ion transmembrane transport, activation of sodium ion membrane transport, activation of sodium ion transmembrane transport Definition: Any process that activates or increases the frequency, rate or extent of sodium ion transmembrane transport. Subtypes: positive regulation of sodium ion export across plasma membrane [GO:1903278], positive regulation of sodium ion import across plasma membrane [GO:1903784], positive regulation of sodium ion transmembrane transporter activity [GO:2000651] Relationships: is a type of positive regulation of sodium ion transport [GO:0010765]; is a type of regulation of sodium ion transmembrane transport [GO:1902305]; is a type of GO:1904064; RO_0002213 sodium ion transmembrane transport [GO:0035725] References: PMID:18591664 Sources: GOC:BHF, GOC:TermGenie, GOC:mtg_cardiac_conduct_nov11, GOC:rl